{
  "term_id": "GO:0007507",
  "term_label": "heart development",
  "gene_name": "Blood vessel epicardial substance",
  "gene_symbol": "BVES",
  "gene": "UniProtKB:Q8NE79"
}